{
  "term_id": "GO:0005737",
  "gene_name": "Proto-oncogene c-Rel",
  "gene": "UniProtKB:Q04864",
  "term_label": "cytoplasm",
  "gene_symbol": "REL"
}